{
  "gene": "UniProtKB:O00321",
  "gene_symbol": "ETV2",
  "gene_name": "ETS translocation variant 2",
  "term_id": "GO:0005634",
  "term_label": "nucleus"
}